{
  "term_label": "cytoplasmic vesicle",
  "gene_name": "Phospholipase D1",
  "gene": "UniProtKB:Q13393",
  "gene_symbol": "PLD1",
  "term_id": "GO:0031410"
}